{
  "term_label": "guanyl-nucleotide exchange factor activity",
  "gene_symbol": "CYTH4",
  "gene": "UniProtKB:Q9UIA0",
  "term_id": "GO:0005085",
  "gene_name": "Cytohesin-4"
}